{
  "gene_symbol": "PPP2R5A",
  "term_id": "UNKNOWN:0001",
  "gene_name": "Serine_threonine-protein phosphatase 2A 56 kDa regulatory subunit alpha isoform",
  "gene": "UniProtKB:Q15172",
  "term_label": "Unknown molecular function"
}